{
  "gene_symbol": "WIPF1",
  "term_id": "GO:0030048",
  "gene_name": "WAS_WASL-interacting protein family member 1",
  "gene": "UniProtKB:O43516",
  "term_label": "actin filament-based movement"
}